{
  "gene_name": "Sodium-coupled neutral amino acid transporter 5",
  "gene": "UniProtKB:Q8WUX1",
  "term_id": "GO:0015186",
  "term_label": "L-glutamine transmembrane transporter activity",
  "gene_symbol": "SLC38A5"
}